ABC-type cadmium transporter activity [GO:0015434] (molecular function) References: PMID:12455987 Definition: Enables the transfer of a solute or solutes from one side of a membrane to the other according to the reaction: ATP + H2O + Cd (cytosol) = ADP + phosphate + Cd (vacuole). Relationships: is a type of cadmium ion transmembrane transporter activity [GO:0015086]; is_a GO:0019829; is a type of ABC-type transporter activity [GO:0140359] Also known as: cadmium ABC transporter, ATP-dependent cadmium transmembrane transporter activity, ATPase-coupled cadmium transmembrane transporter activity, cadmium-transporting ATPase activity